{
  "term_id": "UNKNOWN:0001",
  "gene_name": "Putative UPF0633 protein ENSP00000303136",
  "gene_symbol": "Q5VV11",
  "term_label": "Unknown molecular function",
  "gene": "UniProtKB:Q5VV11"
}